{
  "gene_name": "E-selectin",
  "term_id": "GO:0033691",
  "gene_symbol": "SELE",
  "gene": "UniProtKB:P16581",
  "term_label": "sialic acid binding"
}